{
  "gene": "UniProtKB:Q9BTE3",
  "gene_symbol": "MCMBP",
  "term_label": "chromatin binding",
  "gene_name": "Mini-chromosome maintenance complex-binding protein",
  "term_id": "GO:0003682"
}